{
  "gene_name": "Protein SSX7",
  "gene_symbol": "SSX7",
  "gene": "UniProtKB:Q7RTT5",
  "term_id": "GO:0005634",
  "term_label": "nucleus"
}